negative regulation of glutamate uptake involved in transmission of nerve impulse [GO:0051948] (biological process) Also known as: down regulation of glutamate uptake during transmission of nerve impulse, down-regulation of glutamate uptake during transmission of nerve impulse, downregulation of glutamate uptake during transmission of nerve impulse, negative regulation of glutamate reuptake, inhibition of glutamate uptake during transmission of nerve impulse, negative regulation of glutamate uptake during transmission of nerve impulse, negative regulation of glutamate uptake involved in conduction of nerve impulse Definition: Any process that stops, prevents, or reduces the frequency, rate or extent of the directed movement of L-glutamate into a neuron or glial cell. Relationships: is a type of negative regulation of L-glutamate import across plasma membrane [GO:0002037]; is a type of negative regulation of amino acid uptake involved in synaptic transmission [GO:0051942]; is a type of regulation of glutamate uptake involved in transmission of nerve impulse [GO:0051946]; negatively regulates glutamate reuptake [GO:0051935] Sources: GOC:ai